{
  "term_id": "GO:0007339",
  "gene": "UniProtKB:Q99965",
  "gene_name": "Disintegrin and metalloproteinase domain-containing protein 2",
  "gene_symbol": "ADAM2",
  "term_label": "binding of sperm to zona pellucida"
}